tyramine N-feruloyltransferase activity [GO:0050366] (molecular function) Relationships: is a type of acyltransferase activity, transferring groups other than amino-acyl groups [GO:0016747] Sources: EC:2.3.1.110, MetaCyc:TYRAMINE-N-FERULOYLTRANSFERASE-RXN Also known as: feruloyl-CoA tyramine N-feruloyl-CoA transferase activity, feruloyl-CoA:tyramine N-(hydroxycinnamoyl)transferase activity, feruloyltyramine synthase activity, tyramine N-feruloyl-CoA transferase activity, tyramine feruloyltransferase activity Definition: Catalysis of the reaction: feruloyl-CoA + tyramine = CoA + N-feruloyltyramine.